{
  "gene_symbol": "SATL1",
  "gene": "UniProtKB:Q86VE3",
  "term_id": "GO:0019809",
  "term_label": "spermidine binding",
  "gene_name": "Spermidine_spermine N(1)-acetyltransferase-like protein 1"
}